{
  "gene_symbol": "OR8S1",
  "gene_name": "Olfactory receptor 8S1",
  "term_id": "GO:0005886",
  "term_label": "plasma membrane",
  "gene": "UniProtKB:Q8NH09"
}